{
  "term_label": "response to hypoxia",
  "gene_symbol": "PGF",
  "gene": "UniProtKB:P49763",
  "gene_name": "Placenta growth factor",
  "term_id": "GO:0001666"
}